{
  "gene_symbol": "DEFB126",
  "gene_name": "Beta-defensin 126",
  "gene": "UniProtKB:Q9BYW3",
  "term_id": "UNKNOWN:0001",
  "term_label": "Unknown molecular function"
}